{
  "gene_name": "Lipoyl synthase, mitochondrial",
  "term_id": "GO:0005739",
  "gene_symbol": "LIAS",
  "term_label": "mitochondrion",
  "gene": "UniProtKB:O43766"
}